{
  "gene": "UniProtKB:Q86UD4",
  "term_label": "RNA polymerase II cis-regulatory region sequence-specific DNA binding",
  "term_id": "GO:0000978",
  "gene_name": "Zinc finger protein 329",
  "gene_symbol": "ZNF329"
}